{
  "term_id": "GO:0043015",
  "gene_symbol": "TUBGCP5",
  "gene_name": "Gamma-tubulin complex component 5",
  "gene": "UniProtKB:Q96RT8",
  "term_label": "gamma-tubulin binding"
}